{
  "term_label": "positive regulation of DNA-templated transcription",
  "gene_name": "Myelin regulatory factor-like protein",
  "term_id": "GO:0045893",
  "gene": "UniProtKB:Q96LU7",
  "gene_symbol": "MYRFL"
}